{
  "gene_name": "Olfactory receptor 2T10",
  "gene_symbol": "OR2T10",
  "term_id": "GO:0005886",
  "gene": "UniProtKB:Q8NGZ9",
  "term_label": "plasma membrane"
}